{
  "gene_symbol": "AP2M1",
  "term_label": "clathrin adaptor activity",
  "gene": "UniProtKB:Q96CW1",
  "term_id": "GO:0035615",
  "gene_name": "AP-2 complex subunit mu"
}